{
  "term_label": "COPII-coated ER to Golgi transport vesicle",
  "gene_name": "Endoplasmic reticulum-Golgi intermediate compartment protein 3",
  "term_id": "GO:0030134",
  "gene_symbol": "ERGIC3",
  "gene": "UniProtKB:Q9Y282"
}